{
  "gene_name": "Putative uncharacterized protein encoded by LINC00114",
  "gene": "UniProtKB:Q6XXX2",
  "term_id": "UNKNOWN:0002",
  "term_label": "Unknown biological process",
  "gene_symbol": "LINC00114"
}